{
  "term_id": "GO:0006357",
  "gene_symbol": "NR4A2",
  "term_label": "regulation of transcription by RNA polymerase II",
  "gene_name": "Nuclear receptor subfamily 4 group A member 2",
  "gene": "UniProtKB:P43354"
}